sensitization [GO:0046960] (biological process) Relationships: is a type of GO:0046958 Sources: ISBN:0582227089 Definition: An increased in a behavioral response to a repeated stimulus. For example, a shock to the tail of the marine snail Aplysia, to which the snail responds by withdrawing its gill, will result in increased gill withdrawal the next time the skin is touched.